{
  "gene_symbol": "PRAMEF2",
  "term_id": "GO:0043161",
  "gene": "UniProtKB:O60811",
  "term_label": "proteasome-mediated ubiquitin-dependent protein catabolic process",
  "gene_name": "PRAME family member 2"
}